positive regulation of oxidative stress-induced intrinsic apoptotic signaling pathway [GO:1902177] (biological process) Subtypes: GO:1903378, positive regulation of intrinsic apoptotic signaling pathway in response to hydrogen peroxide [GO:1903752] References: PMID:11672522 Sources: GOC:BHF, GOC:TermGenie, GOC:mtg_apoptosis Also known as: positive regulation of intrinsic apoptotic signaling pathway in response to oxidative stress, up regulation of intrinsic apoptotic signaling pathway in response to oxidative stress, up-regulation of intrinsic apoptotic signaling pathway in response to oxidative stress, upregulation of intrinsic apoptotic signaling pathway in response to oxidative stress, activation of intrinsic apoptotic signaling pathway in response to oxidative stress Definition: Any process that activates or increases the frequency, rate or extent of an oxidative stress-induced intrinsic apoptotic signaling pathway. Relationships: is a type of regulation of oxidative stress-induced intrinsic apoptotic signaling pathway [GO:1902175]; is a type of positive regulation of intrinsic apoptotic signaling pathway [GO:2001244]; positively regulates intrinsic apoptotic signaling pathway in response to oxidative stress [GO:0008631]